{
  "gene_symbol": "NCOR1",
  "term_id": "GO:0003714",
  "term_label": "transcription corepressor activity",
  "gene": "UniProtKB:O75376",
  "gene_name": "Nuclear receptor corepressor 1"
}